{
  "term_id": "UNKNOWN:0002",
  "gene": "UniProtKB:A0A1B0GTS1",
  "term_label": "Unknown biological process",
  "gene_symbol": "HSFX4",
  "gene_name": "Heat shock transcription factor, X-linked member 4"
}